DNA topoisomerase IV complex [GO:0009340] (cellular component) Definition: A heterodimeric enzyme, which in most bacterial species is composed of two subunits, ParC and ParE. Functions in chromosome segregation and can relax supercoiled DNA. References: PMID:7783632 Sources: GOC:jl Relationships: is a type of DNA topoisomerase type II (double strand cut, ATP-hydrolyzing) complex [GO:0009330]